{
  "term_id": "GO:0003729",
  "gene_name": "RNA-binding protein Nova-1",
  "gene": "UniProtKB:P51513",
  "gene_symbol": "NOVA1",
  "term_label": "mRNA binding"
}